{
  "term_label": "cytoplasm",
  "term_id": "GO:0005737",
  "gene_name": "Protein unc-45 homolog B",
  "gene": "UniProtKB:Q8IWX7",
  "gene_symbol": "UNC45B"
}